{
  "term_label": "Unknown molecular function",
  "gene_symbol": "PLK4",
  "gene": "UniProtKB:O00444",
  "gene_name": "Serine_threonine-protein kinase PLK4",
  "term_id": "UNKNOWN:0001"
}